type 2B serotonin receptor binding [GO:0031827] (molecular function) Also known as: 5-hydroxytryptamine 2B receptor binding, type 2B serotonin receptor ligand Relationships: is a type of G protein-coupled serotonin receptor binding [GO:0031821] Definition: Binding to a type 2B serotonin receptor. Sources: GOC:mah, GOC:nln